{
  "gene_symbol": "CDKN2A",
  "gene_name": "Cyclin-dependent kinase inhibitor 2A",
  "term_id": "GO:0008285",
  "gene": "UniProtKB:P42771",
  "term_label": "negative regulation of cell population proliferation"
}